{
  "gene_name": "Phosphatase and actin regulator 2",
  "gene": "UniProtKB:O75167",
  "term_label": "actin binding",
  "term_id": "GO:0003779",
  "gene_symbol": "PHACTR2"
}